symbiont-mediated perturbation of host microtubule cytoskeleton [GO:0141028] (biological process) Definition: The process in which an organism effects a change that impairs the structure or function of the host microtubule cytoskeleton. The host is defined as the larger of the organisms involved in a symbiotic interaction. Also known as: perturbation by symbiont of host microtubule cytoskeleton, disruption by symbiont of host microtubule cytoskeleton, modification by symbiont of host microtubule cytoskeleton Relationships: is_a symbiont-mediated perturbation of host cytoskeleton [GO:0052039] References: PMID:21692747, PMID:26220855